{
  "term_label": "Unknown biological process",
  "term_id": "UNKNOWN:0002",
  "gene": "UniProtKB:P82987",
  "gene_name": "ADAMTS-like protein 3",
  "gene_symbol": "ADAMTSL3"
}